regulation of synoviocyte proliferation [GO:1901645] (biological process) Subtypes: negative regulation of synoviocyte proliferation [GO:1901646], positive regulation of synoviocyte proliferation [GO:1901647] Definition: Any process that modulates the frequency, rate or extent of synoviocyte proliferation. Relationships: is a type of GO:0050678; regulates synoviocyte proliferation [GO:0002941] Sources: GOC:TermGenie